positive regulation of systemic arterial blood pressure [GO:0003084] (biological process) Subtypes: GO:0001982, angiotensin-mediated vasoconstriction involved in regulation of systemic arterial blood pressure [GO:0001998], GO:0002006, vasoconstriction of artery involved in chemoreceptor response to lowering of systemic arterial blood pressure [GO:0002012], vasoconstriction of artery involved in ischemic response to lowering of systemic arterial blood pressure [GO:0002014], regulation of blood volume by renal aldosterone [GO:0002017], negative regulation of renal output by angiotensin [GO:0003083] Relationships: is a type of GO:0045777; is part of regulation of systemic arterial blood pressure [GO:0003073] Definition: The process that increases the force with which blood travels through the systemic arterial circulatory system. Sources: GOC:mtg_cardio